{
  "term_id": "GO:0003729",
  "gene": "UniProtKB:Q8N684",
  "term_label": "mRNA binding",
  "gene_symbol": "CPSF7",
  "gene_name": "Cleavage and polyadenylation specificity factor subunit 7"
}